{
  "term_label": "Unknown biological process",
  "gene_symbol": "PGRMC2",
  "gene": "UniProtKB:O15173",
  "term_id": "UNKNOWN:0002",
  "gene_name": "Membrane-associated progesterone receptor component 2"
}